{
  "gene_name": "Probable ATP-dependent RNA helicase DHX34",
  "gene": "UniProtKB:Q14147",
  "term_label": "RNA binding",
  "term_id": "GO:0003723",
  "gene_symbol": "DHX34"
}